{
  "term_label": "protein serine/threonine kinase activity",
  "term_id": "GO:0004674",
  "gene_name": "Serine_threonine-protein kinase Nek4",
  "gene": "UniProtKB:P51957",
  "gene_symbol": "NEK4"
}